mRNA 3'-end processing by stem-loop binding and cleavage [GO:0006398] (biological process) Definition: Any mRNA 3'-end processing that involves the binding to and cleavage of a stem-loop structure. For example, histone mRNAs contain a highly conserved stem-loop sequence at the 3' end of the mRNA with a 6 base pairs (bp) stem and a 4-nt loop. The mRNA is cleaved between these two elements, after the fourth or fifth nucleotide, which is typically an adenosine. References: PMID:17998288 Sources: GOC:mah, GOC:tb Relationships: is_a histone mRNA metabolic process [GO:0008334]; is a type of GO:0031124 Also known as: histone mRNA 3' end processing